positive regulation of peripheral B cell anergy [GO:0002919] (biological process) Relationships: is a type of positive regulation of peripheral tolerance induction [GO:0002660]; is a type of positive regulation of B cell anergy [GO:0002672]; is a type of GO:0002714; is a type of GO:0002917; positively regulates peripheral B cell anergy [GO:0002453] Definition: Any process that activates or increases the frequency, rate, or extent of peripheral B cell anergy. Sources: GOC:add Also known as: up regulation of peripheral B cell anergy, up-regulation of peripheral B cell anergy, upregulation of peripheral B cell anergy, activation of peripheral B cell anergy, stimulation of peripheral B cell anergy